{
  "term_label": "heparan sulfate proteoglycan catabolic process",
  "term_id": "GO:0030200",
  "gene_symbol": "GUSB",
  "gene_name": "Beta-glucuronidase",
  "gene": "UniProtKB:P08236"
}